{
  "gene_name": "Keratin-associated protein 2-4",
  "term_label": "Unknown cellular component",
  "gene_symbol": "KRTAP2-4",
  "gene": "UniProtKB:Q9BYR9",
  "term_id": "UNKNOWN:0003"
}